{
  "gene_symbol": "SLC12A3",
  "gene": "UniProtKB:P55017",
  "gene_name": "Solute carrier family 12 member 3",
  "term_id": "GO:0035725",
  "term_label": "sodium ion transmembrane transport"
}